{
  "gene_symbol": "OR4C3",
  "term_label": "plasma membrane",
  "term_id": "GO:0005886",
  "gene_name": "Olfactory receptor 4C3",
  "gene": "UniProtKB:Q8NH37"
}